{
  "gene_name": "Cadherin-7",
  "term_label": "cadherin binding",
  "gene": "UniProtKB:Q9ULB5",
  "term_id": "GO:0045296",
  "gene_symbol": "CDH7"
}